glycerol biosynthetic process [GO:0006114] (biological process) Also known as: glycerol anabolism, glycerol biosynthesis, glycerol formation, glycerol synthesis Relationships: is a type of glycerol metabolic process [GO:0006071]; is a type of alditol biosynthetic process [GO:0019401] Sources: GOC:ai, ISBN:0198506732 Subtypes: glycerol biosynthetic process from pyruvate [GO:0046327] Definition: The chemical reactions and pathways resulting in the formation of glycerol, 1,2,3-propanetriol, a sweet, hygroscopic, viscous liquid, widely distributed in nature as a constituent of many lipids.